{
  "term_id": "GO:0000976",
  "term_label": "transcription cis-regulatory region binding",
  "gene": "UniProtKB:Q9BY31",
  "gene_name": "Zinc finger protein 717",
  "gene_symbol": "ZNF717"
}